regulation of mitochondrial membrane permeability involved in programmed necrotic cell death [GO:1902445] (biological process) Definition: Any regulation of mitochondrial membrane permeability that is involved in programmed necrotic cell death. References: PMID:22493254 Sources: GOC:TermGenie, GOC:dph, GOC:mtg_apoptosis Also known as: regulation of transport across mitochondrial membrane involved in programmed necrotic cell death Relationships: is a type of regulation of mitochondrial membrane permeability [GO:0046902]; is part of programmed necrotic cell death [GO:0097300]